{
  "term_label": "nuclear localization sequence binding",
  "gene": "UniProtKB:P52948",
  "term_id": "GO:0008139",
  "gene_symbol": "NUP98",
  "gene_name": "Nuclear pore complex protein Nup98-Nup96"
}